{
  "gene_symbol": "SLC44A3",
  "gene_name": "Choline transporter-like protein 3",
  "gene": "UniProtKB:Q8N4M1",
  "term_label": "membrane",
  "term_id": "GO:0016020"
}